{
  "term_label": "calcium channel regulator activity",
  "gene": "UniProtKB:P55040",
  "gene_name": "GTP-binding protein GEM",
  "term_id": "GO:0005246",
  "gene_symbol": "GEM"
}